antipodal site [GO:0140525] (cellular component) Definition: The pole of the kinetoplast associated with kinetoplast DNA replication. The antipodal sites flank the kinetoplast DNA disk and are positioned approximately 180 degrees apart. In Trypanosoma brucei and Crithidia fasciculata, minicircles are attached at antipodal sites and they contain enzymes that catalyse some of the later reactions in minicircle replication. Relationships: is a type of kinetoplast [GO:0020023] Also known as: antipodal zone References: PMID:12455998, PMID:17462016, PMID:8045928